{
  "term_label": "Unknown cellular component",
  "gene": "UniProtKB:Q6P1R4",
  "term_id": "UNKNOWN:0003",
  "gene_symbol": "DUS1L",
  "gene_name": "tRNA-dihydrouridine(16_17) synthase [NAD(P)(+)]-like"
}